{
  "term_label": "Unknown molecular function",
  "gene": "UniProtKB:Q2TB18",
  "gene_name": "Protein asteroid homolog 1",
  "gene_symbol": "ASTE1",
  "term_id": "UNKNOWN:0001"
}